{
  "gene_name": "Complement C1q and tumor necrosis factor-related protein 9A",
  "gene": "UniProtKB:P0C862",
  "term_label": "Unknown biological process",
  "gene_symbol": "C1QTNF9",
  "term_id": "UNKNOWN:0002"
}